{
  "term_label": "plasma membrane",
  "gene_name": "Olfactory receptor 10G2",
  "gene_symbol": "OR10G2",
  "gene": "UniProtKB:Q8NGC3",
  "term_id": "GO:0005886"
}